{
  "gene": "UniProtKB:Q92973",
  "term_label": "nuclear import signal receptor activity",
  "gene_symbol": "TNPO1",
  "term_id": "GO:0061608",
  "gene_name": "Transportin-1"
}